DSIF complex [GO:0032044] (cellular component) Definition: A heterodimeric protein complex formed of Spt4 and Spt5 proteins which is expressed in eukaryotes from yeast to man. DSIF is an inhibitory elongation factor that promotes RNA polymerase II transcriptional pausing, but can also stimulate transcriptional elongation under certain conditions, and may play a role in RNA processing via its physical association with mRNA capping enzymes. References: PMID:12242279, PMID:12653964, PMID:12676794, PMID:16581788, PMID:19460865 Relationships: is a type of transcription elongation factor complex [GO:0008023] Also known as: 5,6-Dichloro-1-beta-D-ribofuranosylbenzimidazole sensitivity inducing factor complex, DRB sensitivity inducing factor complex, Spt4-Spt5 complex, Spt5-Spt4 complex